{
  "gene": "UniProtKB:P47883",
  "gene_name": "Putative olfactory receptor 3A4",
  "gene_symbol": "OR3A4P",
  "term_id": "GO:0005886",
  "term_label": "plasma membrane"
}